{
  "gene_symbol": "TCP1",
  "term_label": "unfolded protein binding",
  "gene_name": "T-complex protein 1 subunit alpha",
  "term_id": "GO:0051082",
  "gene": "UniProtKB:P17987"
}